{
  "term_id": "GO:0005886",
  "gene_name": "Natural resistance-associated macrophage protein 1",
  "gene_symbol": "SLC11A1",
  "gene": "UniProtKB:P49279",
  "term_label": "plasma membrane"
}